vesicle-mediated cholesterol transport [GO:0090119] (biological process) Relationships: is a type of vesicle-mediated transport [GO:0016192]; is a type of cytosolic transport [GO:0016482]; is a type of intracellular cholesterol transport [GO:0032367] Sources: GOC:ascb_2009, GOC:dph, GOC:tb Definition: The directed movement of cholesterol, cholest-5-en-3-beta-ol, or cholesterol-containing compounds, by membrane-bounded vesicles. Subtypes: endosome to lysosome transport of low-density lipoprotein particle [GO:0090117]